{
  "term_id": "GO:0005886",
  "gene_name": "Growth hormone-regulated TBC protein 1",
  "gene": "UniProtKB:Q5TC63",
  "term_label": "plasma membrane",
  "gene_symbol": "GRTP1"
}